{
  "gene": "UniProtKB:Q8WYP5",
  "term_id": "UNKNOWN:0003",
  "gene_symbol": "AHCTF1",
  "term_label": "Unknown cellular component",
  "gene_name": "Protein ELYS"
}